NuA3a histone acetyltransferase complex [GO:1990467] (cellular component) Relationships: is a type of GO:0033100 References: PMID:25104842 Sources: GOC:rb Definition: A NuA3 complex that catalyzes the acetylation of Histone H3. In S. cerevisiae, this complex consists of Eaf6p, Nto1p, Sas3p, Taf14p, Yng1p and associates with H3K4me3 using Yng1p.